inward migration of deep nuclear neurons [GO:0021948] (BP) Definition: The directed movement of a deep nuclear neuron from the rostrodorsal region of the cerebellar plate to their final more ventral position. Relationships: is a type of neuron migration [GO:0001764]; is_a cell migration in hindbrain [GO:0021535]; BFO_0000050 deep nuclear neuron cell migration [GO:0021946] References: PMID:15157725 Sources: GOC:cls, GOC:dgh, GOC:dph, GOC:jid, GO_REF:0000021